{
  "gene": "UniProtKB:P52739",
  "term_label": "regulation of cytokine production",
  "term_id": "GO:0001817",
  "gene_name": "Zinc finger protein 131",
  "gene_symbol": "ZNF131"
}